negative regulation of SNARE complex disassembly [GO:0035541] (biological process) Relationships: is_a regulation of SNARE complex disassembly [GO:0035495]; is a type of negative regulation of protein-containing complex disassembly [GO:0043242]; is a type of GO:0051051; negatively regulates SNARE complex disassembly [GO:0035494] Definition: Any process that decreases the frequency, rate or extent of disassembly of the SNARE complex. The SNARE complex is a protein complex involved in membrane fusion; a stable ternary complex consisting of a four-helix bundle, usually formed from one R-SNARE and three Q-SNAREs with an ionic layer sandwiched between hydrophobic layers. Sources: GOC:rb